{
  "term_id": "UNKNOWN:0002",
  "gene_symbol": "TRGV1",
  "term_label": "Unknown biological process",
  "gene": "UniProtKB:A0A0A0MS02",
  "gene_name": "Probable non-functional T cell receptor gamma variable"
}